{
  "gene_name": "Clathrin coat assembly protein AP180",
  "term_id": "GO:0008021",
  "gene_symbol": "SNAP91",
  "gene": "UniProtKB:O60641",
  "term_label": "synaptic vesicle"
}